{
  "gene": "UniProtKB:Q05996",
  "gene_name": "Zona pellucida sperm-binding protein 2",
  "gene_symbol": "ZP2",
  "term_label": "acrosin binding",
  "term_id": "GO:0032190"
}